{
  "term_id": "UNKNOWN:0002",
  "gene_symbol": "OR4X1",
  "term_label": "Unknown biological process",
  "gene": "UniProtKB:Q8NH49",
  "gene_name": "Olfactory receptor 4X1"
}